versicolorin B synthase activity [GO:0046572] (molecular function) References: PMID:8784203 Sources: MetaCyc:RXN-9494 Relationships: is a type of carbon-oxygen lyase activity [GO:0016835] Definition: Catalysis of the reaction: versiconal = versicolorin B + H2O.